{
  "gene": "UniProtKB:Q13886",
  "term_label": "DNA-binding transcription factor activity, RNA polymerase II-specific",
  "gene_name": "Krueppel-like factor 9",
  "term_id": "GO:0000981",
  "gene_symbol": "KLF9"
}